{
  "term_label": "Unknown cellular component",
  "gene_symbol": "FNDC9",
  "gene": "UniProtKB:Q8TBE3",
  "term_id": "UNKNOWN:0003",
  "gene_name": "Fibronectin type III domain-containing protein 9"
}